atrazine catabolic process [GO:0019381] (biological process) Relationships: is a type of polyamine catabolic process [GO:0006598]; is_a s-triazine compound catabolic process [GO:0042204]; is a type of organohalogen metabolic process [GO:0090345] Sources: GOC:jl, MetaCyc:PWY-5724 Subtypes: atrazine catabolic process to urea [GO:0019623], atrazine catabolic process to isopropylamine [GO:0019624], GO:0019625 Also known as: atrazine breakdown, atrazine catabolism, atrazine degradation Definition: The chemical reactions and pathways resulting in the breakdown of atrazine, a triazine ring-containing herbicide.